negative regulation of viral genome replication [GO:0045071] (biological process) Relationships: is_a GO:0045069; is a type of negative regulation of viral process [GO:0048525]; negatively regulates viral genome replication [GO:0019079] Subtypes: negative regulation of single stranded viral RNA replication via double stranded DNA intermediate [GO:0045869] Sources: GOC:go_curators Also known as: down regulation of viral genome replication, down-regulation of viral genome replication, downregulation of viral genome replication, inhibition of viral genome replication Definition: Any process that stops, prevents, or reduces the frequency, rate or extent of viral genome replication.